regulation of mesodermal cell fate determination [GO:0048334] (biological process) Relationships: is a type of GO:1905770; is_a GO:1905933; is a type of regulation of animal organ morphogenesis [GO:2000027]; regulates GO:0007500 Definition: Any process that modulates the frequency, rate or extent of mesoderm cell fate determination. Sources: GOC:dgh Subtypes: regulation of axial mesodermal cell fate determination [GO:0048324], GO:0048335, positive regulation of mesodermal cell fate determination [GO:0048336], regulation of paraxial mesodermal cell fate determination [GO:0048345], regulation of lateral mesodermal cell fate determination [GO:0048374], regulation of intermediate mesodermal cell fate determination [GO:0048395]